{
  "gene_name": "C-U-editing enzyme APOBEC-1",
  "term_id": "GO:0005634",
  "gene": "UniProtKB:P41238",
  "term_label": "nucleus",
  "gene_symbol": "APOBEC1"
}